{
  "gene_name": "Tumor necrosis factor ligand superfamily member 10",
  "term_label": "extracellular space",
  "gene": "UniProtKB:P50591",
  "term_id": "GO:0005615",
  "gene_symbol": "TNFSF10"
}